{
  "gene_name": "Kelch-like protein 3",
  "term_id": "GO:0005737",
  "gene_symbol": "KLHL3",
  "gene": "UniProtKB:Q9UH77",
  "term_label": "cytoplasm"
}